{
  "term_id": "GO:0001675",
  "term_label": "acrosome assembly",
  "gene": "UniProtKB:P52594",
  "gene_symbol": "AGFG1",
  "gene_name": "Arf-GAP domain and FG repeat-containing protein 1"
}